{
  "term_label": "positive regulation of transcription by RNA polymerase II",
  "gene_name": "Insulin gene enhancer protein ISL-2",
  "term_id": "GO:0045944",
  "gene_symbol": "ISL2",
  "gene": "UniProtKB:Q96A47"
}